{
  "gene_name": "Dolichyl-phosphate beta-glucosyltransferase",
  "gene": "UniProtKB:Q9Y673",
  "gene_symbol": "ALG5",
  "term_id": "GO:0005789",
  "term_label": "endoplasmic reticulum membrane"
}